{
  "gene_symbol": "LZTFL1",
  "term_id": "GO:0005929",
  "gene": "UniProtKB:Q9NQ48",
  "term_label": "cilium",
  "gene_name": "Leucine zipper transcription factor-like protein 1"
}